negative regulation of amoeboid sperm motility [GO:1905417] (biological process) Definition: Any process that stops, prevents or reduces the frequency, rate or extent of amoeboid sperm motility. Also known as: down regulation of ameboid sperm motility, down regulation of ameboid sperm movement, down regulation of amoeboid sperm motility, down regulation of amoeboid sperm movement, down-regulation of ameboid sperm motility, down-regulation of ameboid sperm movement, down-regulation of amoeboid sperm motility, down-regulation of amoeboid sperm movement, downregulation of ameboid sperm motility, downregulation of ameboid sperm movement, downregulation of amoeboid sperm motility, downregulation of amoeboid sperm movement, negative regulation of ameboid sperm motility, negative regulation of ameboid sperm movement, negative regulation of amoeboid sperm movement, inhibition of ameboid sperm motility, inhibition of ameboid sperm movement, inhibition of amoeboid sperm motility, inhibition of amoeboid sperm movement Sources: GOC:TermGenie, GOC:cilia, GOC:krc, GO_REF:0000058 Relationships: is a type of regulation of amoeboid sperm motility [GO:1905416]; is a type of negative regulation of cell motility [GO:2000146]; is a type of negative regulation of reproductive process [GO:2000242]; RO_0002212 amoeboid sperm motility [GO:0097723]